{
  "term_id": "GO:0005739",
  "gene_name": "Aconitate hydratase, mitochondrial",
  "gene": "UniProtKB:Q99798",
  "gene_symbol": "ACO2",
  "term_label": "mitochondrion"
}